mesonephric cell migration involved in male gonad development [GO:0061457] (biological process) Relationships: is a type of cell migration [GO:0016477] Definition: The orderly movement of a cell from the mesonephros to the male gonad, contributing to its development. Sources: GOC:dph, GOC:tb